metanephric macula densa development [GO:0072227] (BP) Sources: GOC:mtg_kidney_jan10 Relationships: is a type of GO:0072024; is a type of metanephric nephron epithelium development [GO:0072243]; BFO_0000050 GO:0072206 Definition: The process whose specific outcome is the progression of the metanephric macula densa over time, from its formation to the mature structure. The metanephric macula densa is an area of specialized cells in the distal tubule of the metanephros that makes contact with the vascular pole of the glomerulus.